{
  "gene_symbol": "ATIC",
  "gene_name": "Bifunctional purine biosynthesis protein ATIC",
  "gene": "UniProtKB:P31939",
  "term_id": "GO:0005829",
  "term_label": "cytosol"
}